{
  "gene": "UniProtKB:Q9UPN4",
  "term_label": "Unknown molecular function",
  "gene_symbol": "CEP131",
  "gene_name": "Centrosomal protein of 131 kDa",
  "term_id": "UNKNOWN:0001"
}